{
  "term_id": "GO:0005886",
  "gene_name": "Oxysterol-binding protein-related protein 6",
  "gene": "UniProtKB:Q9BZF3",
  "term_label": "plasma membrane",
  "gene_symbol": "OSBPL6"
}